choline:oxygen 1-oxidoreductase activity [GO:0033713] (molecular function) Relationships: is_a oxidoreductase activity, acting on the CH-OH group of donors, oxygen as acceptor [GO:0016899] Sources: EC:1.1.3.17, RHEA:13505 Definition: Catalysis of the reaction: choline + O2 = betaine aldehyde + hydrogen peroxide. Also known as: choline oxidase activity